isopentenyl pyrophosphate import into mitochondrion [GO:0170046] (biological process) Relationships: is a type of organic anion transport [GO:0015711]; is a type of GO:0015914; is a type of intracellular lipid transport [GO:0032365]; is a type of import into the mitochondrion [GO:0170036] References: PMID:37813972 Sources: GOC:ew Definition: The process in which isopentenyl pyrophosphate is transported across a membrane into the mitochondrion.